protein arginine kinase activity [GO:1990424] (molecular function) Definition: Catalysis of the reaction: ATP + a protein arginine = ADP + protein arginine phosphate. Note: This reaction occurs in bacterial species e.g. Bacillus subtilis. Relationships: is a type of protein kinase activity [GO:0004672] References: PMID:22517742 Sources: RHEA:43384 Also known as: protein-arginine kinase activity